{
  "gene_symbol": "ZNF365",
  "gene": "UniProtKB:Q70YC5",
  "term_label": "Unknown cellular component",
  "gene_name": "Protein ZNF365",
  "term_id": "UNKNOWN:0003"
}